{
  "term_id": "GO:0005634",
  "gene_name": "Zinc finger protein with KRAB and SCAN domains 7",
  "gene_symbol": "ZKSCAN7",
  "term_label": "nucleus",
  "gene": "UniProtKB:Q9P0L1"
}